{
  "term_id": "GO:0016477",
  "gene": "UniProtKB:P08134",
  "term_label": "cell migration",
  "gene_name": "Rho-related GTP-binding protein RhoC",
  "gene_symbol": "RHOC"
}